{
  "term_label": "extracellular space",
  "gene_name": "Matrix metalloproteinase-28",
  "term_id": "GO:0005615",
  "gene_symbol": "MMP28",
  "gene": "UniProtKB:Q9H239"
}